{
  "gene_symbol": "DHRS9",
  "gene_name": "Dehydrogenase_reductase SDR family member 9",
  "term_label": "steroid metabolic process",
  "gene": "UniProtKB:Q9BPW9",
  "term_id": "GO:0008202"
}